positive regulation of naphtho-gamma-pyrone biosynthetic process [GO:1900848] (BP) Definition: Any process that activates or increases the frequency, rate or extent of naphtho-gamma-pyrone biosynthetic process. Also known as: up regulation of naphtho-gamma-pyrone biosynthetic process, up-regulation of naphtho-gamma-pyrone biosynthetic process, upregulation of naphtho-gamma-pyrone biosynthetic process, activation of naphtho-gamma-pyrone biosynthetic process Sources: GOC:TermGenie, GOC:di Relationships: is a type of positive regulation of biosynthetic process [GO:0009891]; is a type of positive regulation of small molecule metabolic process [GO:0062013]; is a type of regulation of naphtho-gamma-pyrone biosynthetic process [GO:1900846]; positively regulates naphtho-gamma-pyrone biosynthetic process [GO:1900787]